{
  "term_id": "UNKNOWN:0001",
  "gene_name": "Uncharacterized protein C6orf141",
  "gene_symbol": "C6orf141",
  "term_label": "Unknown molecular function",
  "gene": "UniProtKB:Q5SZD1"
}